{
  "term_label": "phagocytosis, engulfment",
  "gene_symbol": "HAVCR1",
  "term_id": "GO:0006911",
  "gene": "UniProtKB:Q96D42",
  "gene_name": "Hepatitis A virus cellular receptor 1"
}